{
  "term_label": "positive regulation of MAPK cascade",
  "gene_symbol": "LAMTOR1",
  "gene": "UniProtKB:Q6IAA8",
  "gene_name": "Ragulator complex protein LAMTOR1",
  "term_id": "GO:0043410"
}